{
  "gene_symbol": "RAB13",
  "term_label": "endosome",
  "term_id": "GO:0005768",
  "gene_name": "Ras-related protein Rab-13",
  "gene": "UniProtKB:P51153"
}